{
  "gene_name": "Alpha-1,3-mannosyl-glycoprotein 4-beta-N-acetylglucosaminyltransferase B",
  "gene_symbol": "MGAT4B",
  "term_label": "endoplasmic reticulum-Golgi intermediate compartment",
  "term_id": "GO:0005793",
  "gene": "UniProtKB:Q9UQ53"
}